{
  "term_id": "GO:0005634",
  "gene_symbol": "PPARGC1A",
  "gene_name": "Peroxisome proliferator-activated receptor gamma coactivator 1-alpha",
  "term_label": "nucleus",
  "gene": "UniProtKB:Q9UBK2"
}